{
  "gene": "UniProtKB:A0ZSE6",
  "term_id": "UNKNOWN:0002",
  "term_label": "Unknown biological process",
  "gene_symbol": "TMEM30CP",
  "gene_name": "Cell cycle control protein 50C"
}